response to oxygen levels [GO:0070482] (biological process) Sources: GOC:BHF, GOC:mah Definition: Any process that results in a change in state or activity of a cell or an organism (in terms of movement, secretion, enzyme production, gene expression, etc.) as a result of a stimulus reflecting the presence, absence, or concentration of oxygen. Subtypes: detection of oxygen [GO:0003032], response to decreased oxygen levels [GO:0036293], GO:0036296, cellular response to oxygen levels [GO:0071453] Relationships: is a type of response to abiotic stimulus [GO:0009628]